{
  "term_label": "receptor ligand activity",
  "gene": "UniProtKB:Q8WWG1",
  "term_id": "GO:0048018",
  "gene_symbol": "NRG4",
  "gene_name": "Pro-neuregulin-4, membrane-bound isoform"
}